regulation of cellular response to testosterone stimulus [GO:2000654] (biological process) Subtypes: GO:2000655 Definition: Any process that modulates the frequency, rate or extent of cellular response to testosterone stimulus. Relationships: is a type of GO:0048583; is_a regulation of cellular process [GO:0050794]; regulates cellular response to testosterone stimulus [GO:0071394] Sources: GOC:BHF